{
  "term_label": "cell differentiation",
  "gene_symbol": "FSTL3",
  "gene_name": "Follistatin-related protein 3",
  "gene": "UniProtKB:O95633",
  "term_id": "GO:0030154"
}